{
  "term_label": "endoplasmic reticulum",
  "gene_name": "Transmembrane emp24 domain-containing protein 10",
  "gene_symbol": "TMED10",
  "gene": "UniProtKB:P49755",
  "term_id": "GO:0005783"
}